{
  "gene_symbol": "COMMD2",
  "term_id": "UNKNOWN:0001",
  "term_label": "Unknown molecular function",
  "gene": "UniProtKB:Q86X83",
  "gene_name": "COMM domain-containing protein 2"
}